{
  "gene_name": "CXXC-type zinc finger protein 5",
  "term_id": "GO:0005634",
  "gene": "UniProtKB:Q7LFL8",
  "gene_symbol": "CXXC5",
  "term_label": "nucleus"
}